{
  "gene_symbol": "SUOX",
  "gene": "UniProtKB:P51687",
  "term_label": "sulfur compound metabolic process",
  "term_id": "GO:0006790",
  "gene_name": "Sulfite oxidase, mitochondrial"
}